ketotetrose-phosphate aldolase activity [GO:0050014] (molecular function) Relationships: is a type of aldehyde-lyase activity [GO:0016832] Sources: EC:4.1.2.2, RHEA:20932 Definition: Catalysis of the reaction: L-erythrulose 1-phosphate = formaldehyde + glycerone phosphate. Also known as: erythrose-1-phosphate synthase activity, erythrulose-1-phosphate formaldehyde-lyase (glycerone-phosphate-forming), erythrulose-1-phosphate formaldehyde-lyase activity, erythrulose-1-phosphate synthetase activity, phosphoketotetrose aldolase activity